{
  "gene_name": "Chloride anion exchanger",
  "term_id": "GO:0015116",
  "term_label": "sulfate transmembrane transporter activity",
  "gene_symbol": "SLC26A3",
  "gene": "UniProtKB:P40879"
}